{
  "gene_symbol": "CATR1",
  "gene": "UniProtKB:Q13166",
  "term_id": "UNKNOWN:0003",
  "gene_name": "CATR tumorigenic conversion 1 protein",
  "term_label": "Unknown cellular component"
}